{
  "gene_name": "Armadillo repeat-containing protein 10",
  "gene": "UniProtKB:Q8N2F6",
  "gene_symbol": "ARMC10",
  "term_label": "Unknown molecular function",
  "term_id": "UNKNOWN:0001"
}